{
  "term_id": "GO:0061061",
  "gene": "UniProtKB:Q53GG5",
  "term_label": "muscle structure development",
  "gene_name": "PDZ and LIM domain protein 3",
  "gene_symbol": "PDLIM3"
}